{
  "gene": "UniProtKB:Q00839",
  "term_label": "nucleus",
  "term_id": "GO:0005634",
  "gene_name": "Heterogeneous nuclear ribonucleoprotein U",
  "gene_symbol": "HNRNPU"
}